phosphoglucan, water dikinase activity [GO:0051752] (molecular function) Also known as: ATP:phospho-alpha-glucan, water phosphotransferase activity, OK1, PWD Definition: Catalysis of the reaction: [(1->4)-6-phospho-alpha-D-glucosyl](n) + n ATP + n H2O = [(1->4)-3,6-bisphospho-alpha-alpha-glucosyl](n) + n AMP + 2n H+ + n phosphate. References: PMID:15618411 Sources: RHEA:10256 Relationships: is a type of kinase activity [GO:0016301]; is a type of phosphotransferase activity, paired acceptors [GO:0016781]